endonucleolytic cleaveage between SSU-rRNA and LSU-rRNA of tetracistronic rRNA transcript (SSU-rRNA, LSU-rRNA, 4.5S-rRNA, 5S-rRNA) [GO:0002106] (BP) Definition: Endonucleolytic cleavages between the SSU-rRNA and the LSU-rRNA of an rRNA molecule originally produced as a tetracistronic rRNA transcript that contains the Small Subunit (SSU) rRNA, Large Subunit (LSU) the 4.5S rRNA, and the 5S rRNA in that order from 5' to 3' along the primary transcript. These cleavages liberate tRNAs from the polycistronic transcript as well as separating the SSU and LSU containing transcript. Note that the use of the word tetracistronic refers only to the number of mature rRNA molecules which will be produced from the primary transcript and ignores tRNAs that may also be present within the primary transcript. Relationships: is a type of endonucleolytic cleavage of tetracistronic rRNA transcript (SSU-rRNA, LSU-rRNA, 4.5S-rRNA, 5S-rRNA) [GO:0002103] Sources: GOC:curators